{
  "gene_symbol": "SCN2B",
  "term_id": "GO:0061337",
  "term_label": "cardiac conduction",
  "gene_name": "Sodium channel subunit beta-2",
  "gene": "UniProtKB:O60939"
}